{
  "gene": "UniProtKB:Q6ZTQ4",
  "gene_symbol": "CDHR3",
  "term_id": "GO:0007043",
  "gene_name": "Cadherin-related family member 3",
  "term_label": "cell-cell junction assembly"
}